{
  "term_id": "GO:0006357",
  "gene_name": "Homeobox protein Hox-A11",
  "gene": "UniProtKB:P31270",
  "gene_symbol": "HOXA11",
  "term_label": "regulation of transcription by RNA polymerase II"
}